lyase activity [GO:0016829] (molecular function) Regulation: positively regulated by positive regulation of lyase activity [GO:0051349] Subtypes: ferrochelatase activity [GO:0004325], carbon-carbon lyase activity [GO:0016830], GO:0016835, GO:0016840, carbon-sulfur lyase activity [GO:0016846], carbon-halide lyase activity [GO:0016848], phosphorus-oxygen lyase activity [GO:0016849], GO:0016852, GO:0018835, GO:0018836, 3'-deoxyribose phosphate lyase activity [GO:0106334], nitrogen-oxygen lyase activity [GO:0141122], GO:0160129 Sources: EC:4.-.-.- Relationships: is a type of GO:0003824 Definition: Catalysis of the cleavage of C-C, C-O, C-N and other bonds by other means than by hydrolysis or oxidation, or conversely adding a group to a double bond. They differ from other enzymes in that two substrates are involved in one reaction direction, but only one in the other direction. When acting on the single substrate, a molecule is eliminated and this generates either a new double bond or a new ring.